{
  "term_label": "microvillus organization",
  "gene": "UniProtKB:Q8N271",
  "term_id": "GO:0032528",
  "gene_symbol": "PROM2",
  "gene_name": "Prominin-2"
}